regulation of cell wall organization or biogenesis [GO:1903338] (biological process) Definition: Any process that modulates the frequency, rate or extent of cell wall organization or biogenesis. Subtypes: regulation of fungal-type cell wall biogenesis [GO:0032995], regulation of fungal-type cell wall organization [GO:0060237], regulation of plant-type cell wall organization or biogenesis [GO:0080157], GO:0090334, GO:1903339, GO:1903340, GO:2000652 Relationships: is a type of regulation of cellular process [GO:0050794]; regulates cell wall organization or biogenesis [GO:0071554] Sources: GOC:TermGenie, GOC:vw, GO_REF:0000058 Also known as: regulation of cell wall organisation or biogenesis, regulation of cell wall organization or biogenesis at cellular level, regulation of cellular cell wall organisation or biogenesis, regulation of cellular cell wall organization or biogenesis